{
  "term_label": "signaling receptor binding",
  "gene_name": "Putative butyrophilin subfamily 2 member A3",
  "gene_symbol": "BTN2A3P",
  "gene": "UniProtKB:Q96KV6",
  "term_id": "GO:0005102"
}